{
  "gene_name": "Soluble calcium-activated nucleotidase 1",
  "gene_symbol": "CANT1",
  "term_label": "Unknown cellular component",
  "term_id": "UNKNOWN:0003",
  "gene": "UniProtKB:Q8WVQ1"
}